{
  "gene_name": "Sodium-dependent serotonin transporter",
  "term_id": "GO:0005886",
  "term_label": "plasma membrane",
  "gene_symbol": "SLC6A4",
  "gene": "UniProtKB:P31645"
}